{
  "gene_symbol": "PARP14",
  "gene_name": "Protein mono-ADP-ribosyltransferase PARP14",
  "term_id": "GO:0005737",
  "term_label": "cytoplasm",
  "gene": "UniProtKB:Q460N5"
}